{
  "gene_symbol": "CYP1A1",
  "term_id": "GO:0006706",
  "gene": "UniProtKB:P04798",
  "term_label": "steroid catabolic process",
  "gene_name": "Cytochrome P450 1A1"
}